{
  "term_id": "UNKNOWN:0003",
  "gene_symbol": "NDUFS1",
  "gene": "UniProtKB:P28331",
  "gene_name": "NADH-ubiquinone oxidoreductase 75 kDa subunit, mitochondrial",
  "term_label": "Unknown cellular component"
}